{
  "gene_name": "Immunoglobulin superfamily member 21",
  "term_label": "presynaptic membrane",
  "gene_symbol": "IGSF21",
  "gene": "UniProtKB:Q96ID5",
  "term_id": "GO:0042734"
}